skeletal muscle regeneration at neuromuscular junction [GO:0014730] (BP) Definition: The regrowth of muscle tissue to repair injured or damaged muscle fibers in the postnatal stage at the neuromuscular junction. Regeneration of neuromuscular junctions occurs in an orderly way and relies on communication between nerve and muscle. Skeletal myofibers regenerate after injury and form neuro-muscular junctions with motor axons similar to normal ones. Regenerating myofibers develop within the basal lamina sheaths (satellite cells) of original myofibers. Sources: GOC:mtg_muscle Relationships: is a type of skeletal muscle tissue regeneration [GO:0043403]